response to gold nanoparticle [GO:1990268] (biological process) References: PMID:23150627 Relationships: is a type of GO:1990267 Definition: Any process that results in a change in state or activity of a cell or an organism (in terms of movement, secretion, enzyme production, gene expression, etc.) as a result of a gold nanoparticle stimulus.